{
  "gene": "UniProtKB:O95498",
  "term_label": "Unknown cellular component",
  "gene_name": "Pantetheine hydrolase VNN2",
  "gene_symbol": "VNN2",
  "term_id": "UNKNOWN:0003"
}